{
  "term_label": "positive regulation of cell migration",
  "gene": "UniProtKB:Q05397",
  "gene_symbol": "PTK2",
  "gene_name": "Focal adhesion kinase 1",
  "term_id": "GO:0030335"
}